tumor necrosis factor receptor superfamily complex [GO:0002947] (cellular component) Also known as: TNF receptor superfamily complex Sources: GOC:krc Definition: A receptor complex that contains one or more members of the tumor necrosis factor (TNF) receptor superfamily. Relationships: is a type of GO:0043235